{
  "term_id": "GO:0001228",
  "term_label": "DNA-binding transcription activator activity, RNA polymerase II-specific",
  "gene_name": "Cyclic AMP-dependent transcription factor ATF-4",
  "gene_symbol": "ATF4",
  "gene": "UniProtKB:P18848"
}